{
  "gene_symbol": "ZSCAN29",
  "gene_name": "Zinc finger and SCAN domain-containing protein 29",
  "gene": "UniProtKB:Q8IWY8",
  "term_label": "regulation of transcription by RNA polymerase II",
  "term_id": "GO:0006357"
}